{
  "term_label": "cell surface",
  "term_id": "GO:0009986",
  "gene_symbol": "ITGB8",
  "gene": "UniProtKB:P26012",
  "gene_name": "Integrin beta-8"
}